cellular detoxification of cadmium ion [GO:0098849] (biological process) Relationships: is a type of GO:0071585; is a type of GO:0140961; is part of cellular response to cadmium ion [GO:0071276] Sources: GOC:dos, GOC:vw Definition: Any process that reduces or removes the toxicity of cadmium cations in a cell. These include transport of cadmium cations away from sensitive areas and to compartments or complexes whose purpose is sequestration.